{
  "term_label": "Unknown cellular component",
  "gene_symbol": "C3orf80",
  "term_id": "UNKNOWN:0003",
  "gene_name": "Uncharacterized membrane protein C3orf80",
  "gene": "UniProtKB:F5H4A9"
}